{
  "term_id": "GO:0016176",
  "gene_symbol": "NCF1",
  "gene": "UniProtKB:P14598",
  "term_label": "superoxide-generating NADPH oxidase activator activity",
  "gene_name": "Neutrophil cytosol factor 1"
}